{
  "gene_symbol": "KCNH4",
  "gene": "UniProtKB:Q9UQ05",
  "gene_name": "Potassium voltage-gated channel subfamily H member 4",
  "term_label": "voltage-gated potassium channel activity",
  "term_id": "GO:0005249"
}